{
  "gene_symbol": "DTNBP1",
  "gene_name": "Dysbindin",
  "term_label": "regulation of signal transduction",
  "term_id": "GO:0009966",
  "gene": "UniProtKB:Q96EV8"
}